{
  "gene_name": "Solute carrier family 22 member 17",
  "term_id": "UNKNOWN:0002",
  "gene_symbol": "SLC22A17",
  "term_label": "Unknown biological process",
  "gene": "UniProtKB:Q8WUG5"
}